{
  "term_id": "GO:0005886",
  "gene_name": "Protein EFR3 homolog B",
  "term_label": "plasma membrane",
  "gene": "UniProtKB:Q9Y2G0",
  "gene_symbol": "EFR3B"
}